pyrimidine nucleotide interconversion [GO:0015953] (biological process) Sources: GOC:mah, ISBN:0306444747, ISBN:0471394831 Subtypes: GO:0015954, GO:0015955 Relationships: is_a pyrimidine nucleotide metabolic process [GO:0006220]; is a type of nucleobase-containing small molecule interconversion [GO:0015949] Definition: The chemical reactions and pathways by which a pyrimidine nucleotide is synthesized from another pyrimidine nucleotide.